{
  "gene": "UniProtKB:P41440",
  "gene_symbol": "SLC19A1",
  "gene_name": "Reduced folate transporter",
  "term_id": "GO:0005542",
  "term_label": "folic acid binding"
}